{
  "gene_name": "Protein kinase C eta type",
  "term_label": "Unknown cellular component",
  "term_id": "UNKNOWN:0003",
  "gene_symbol": "PRKCH",
  "gene": "UniProtKB:P24723"
}